{
  "gene_name": "Caspase recruitment domain-containing protein 11",
  "term_label": "cytoplasm",
  "gene_symbol": "CARD11",
  "gene": "UniProtKB:Q9BXL7",
  "term_id": "GO:0005737"
}